{
  "gene_name": "Zinc finger protein 827",
  "gene": "UniProtKB:Q17R98",
  "gene_symbol": "ZNF827",
  "term_id": "GO:0003700",
  "term_label": "DNA-binding transcription factor activity"
}